{
  "term_id": "GO:0036402",
  "gene": "UniProtKB:P17980",
  "gene_name": "26S proteasome regulatory subunit 6A",
  "gene_symbol": "PSMC3",
  "term_label": "proteasome-activating activity"
}